{
  "term_label": "Unknown cellular component",
  "gene": "UniProtKB:Q13237",
  "term_id": "UNKNOWN:0003",
  "gene_name": "cGMP-dependent protein kinase 2",
  "gene_symbol": "PRKG2"
}